{
  "term_id": "GO:0005634",
  "term_label": "nucleus",
  "gene_symbol": "LGALS9B",
  "gene_name": "Galectin-9B",
  "gene": "UniProtKB:Q3B8N2"
}